peroxynitrite isomerase activity [GO:0062213] (molecular function) Definition: Catalysis of the reaction: peroxynitrite = nitrate. References: PMID:30524950 Sources: RHEA:63116 Relationships: is a type of isomerase activity [GO:0016853]